{
  "term_id": "UNKNOWN:0001",
  "gene_name": "Melanoma-associated antigen B1",
  "term_label": "Unknown molecular function",
  "gene": "UniProtKB:P43366",
  "gene_symbol": "MAGEB1"
}